{
  "term_label": "presynaptic active zone",
  "gene_symbol": "GAD1",
  "term_id": "GO:0048786",
  "gene": "UniProtKB:Q99259",
  "gene_name": "Glutamate decarboxylase 1"
}